{
  "gene_symbol": "SPEM2",
  "term_label": "Unknown biological process",
  "gene_name": "Uncharacterized protein SPEM2",
  "gene": "UniProtKB:Q0P670",
  "term_id": "UNKNOWN:0002"
}